integrin alphaL-beta2 complex [GO:0034687] (cellular component) Definition: An integrin complex that comprises one alphaL subunit and one beta2 subunit. Also known as: alphaL-beta2 integrin complex, Itgal-Itgb2 complex Relationships: is a type of GO:0008305 References: PMID:12297042